{
  "gene_name": "Uncharacterized protein C9orf153",
  "gene_symbol": "C9orf153",
  "term_label": "Unknown biological process",
  "gene": "UniProtKB:Q5TBE3",
  "term_id": "UNKNOWN:0002"
}